new growing cell tip [GO:0035841] (cellular component) Definition: A cell tip that was newly formed at the last cell division, and that has started to grow after the cell has activated bipolar cell growth (i.e. in which new end take-off, NETO, has taken place). New end take-off is when monopolar cells initiate bipolar growth. References: PMID:19431238 Sources: GOC:expert_jd, GOC:mah Relationships: is a type of growing cell tip [GO:0035838] Also known as: new cell tip after activation of bipolar cell growth, post-NETO new cell end, post-NETO new cell tip, post-new end take-off new cell tip